{
  "gene_name": "Zinc finger protein castor homolog 1",
  "gene_symbol": "CASZ1",
  "gene": "UniProtKB:Q86V15",
  "term_id": "GO:0005634",
  "term_label": "nucleus"
}